{
  "term_id": "GO:0005886",
  "gene_name": "NKG2-A_NKG2-B type II integral membrane protein",
  "term_label": "plasma membrane",
  "gene_symbol": "KLRC1",
  "gene": "UniProtKB:P26715"
}